eye pigment metabolic process [GO:0042441] (biological process) Definition: The chemical reactions and pathways involving eye pigments, any general or particular coloring matter in living organisms, found or utilized in the eye. Sources: GOC:ai Also known as: eye pigment metabolism Relationships: is a type of pigment metabolic process involved in developmental pigmentation [GO:0043324]; is part of eye pigmentation [GO:0048069] Subtypes: eye pigment biosynthetic process [GO:0006726], GO:0046151, ommochrome metabolic process [GO:0046152], rhodopsin metabolic process [GO:0046154]